{
  "term_id": "UNKNOWN:0001",
  "gene_symbol": "C22orf31",
  "term_label": "Unknown molecular function",
  "gene_name": "Uncharacterized protein C22orf31",
  "gene": "UniProtKB:O95567"
}